{
  "gene_name": "CYFIP-related Rac1 interactor B",
  "term_label": "Unknown molecular function",
  "term_id": "UNKNOWN:0001",
  "gene": "UniProtKB:Q9NUQ9",
  "gene_symbol": "CYRIB"
}